{
  "gene_name": "Gamma-aminobutyric acid receptor subunit gamma-2",
  "gene": "UniProtKB:P18507",
  "term_id": "GO:0098794",
  "gene_symbol": "GABRG2",
  "term_label": "postsynapse"
}